histone H3K9 acetyltransferase activity [GO:0043992] (MF) References: PMID:18552846, PMID:19056256 Note: Comment: Note that the residue position corresponds to the canonical human H3 histone (UniProtKB:P84243); this residue is conserved across all eukaryotes. Residue 1 is the first residue following removal of the initiating Methionine (Met). Note that each histone is encoded by multiple genes, and sequences may vary across different genes within an organism. Definition: Catalysis of the reaction: acetyl-CoA + histone H3 L-lysine (position 9) = CoA + histone H3 N6-acetyl-L-lysine (position 9). Relationships: is a type of histone H3 acetyltransferase activity [GO:0010484] Also known as: histone H3-K9 acetyltransferase activity, histone acetylase activity (H3-K9 specific), histone acetyltransferase activity (H3-K9 specific), histone lysine N-acetyltransferase activity (H3-K9 specific)